{
  "gene_name": "Uncharacterized protein DKFZp434B061",
  "term_id": "UNKNOWN:0001",
  "term_label": "Unknown molecular function",
  "gene_symbol": "Q9UF83",
  "gene": "UniProtKB:Q9UF83"
}